regulation of actin filament depolymerization [GO:0030834] (biological process) Sources: GOC:mah Definition: Any process that modulates the frequency, rate or extent of the disassembly of actin filaments by the removal of actin monomers from a filament. Also known as: regulation of actin depolymerization Relationships: is_a regulation of actin polymerization or depolymerization [GO:0008064]; is a type of GO:1901879; regulates GO:0030042 Subtypes: negative regulation of actin filament depolymerization [GO:0030835], positive regulation of actin filament depolymerization [GO:0030836], GO:2000812